{
  "term_label": "Unknown molecular function",
  "gene": "UniProtKB:Q8NA31",
  "gene_name": "Telomere repeats-binding bouquet formation protein 1",
  "term_id": "UNKNOWN:0001",
  "gene_symbol": "TERB1"
}